disruption of cell in another organism [GO:0141061] (biological process) Definition: The disruption of a cell of another organism, leading to damage or temporary subversion of that cell. Sources: GOC:pg Relationships: is a type of disruption of anatomical structure in another organism [GO:0141060] Subtypes: killing of cells of another organism [GO:0031640]